macromolecule methylation [GO:0043414] (biological process) Relationships: is a type of methylation [GO:0032259]; is a type of macromolecule modification [GO:0043412] Subtypes: GO:0001510, protein methylation [GO:0006479] Definition: The covalent attachment of a methyl residue to one or more monomeric units in a polypeptide, polynucleotide, polysaccharide, or other biological macromolecule. Sources: GOC:go_curators